positive regulation of acetylcholine secretion, neurotransmission [GO:0014057] (biological process) Also known as: up regulation of acetylcholine secretion, up-regulation of acetylcholine secretion, upregulation of acetylcholine secretion, activation of acetylcholine secretion, stimulation of acetylcholine secretion Definition: Any process that activates or increases the frequency, rate or extent of the regulated release of acetylcholine. Relationships: is a type of positive regulation of neurotransmitter secretion [GO:0001956]; is a type of regulation of acetylcholine secretion, neurotransmission [GO:0014056]; is a type of positive regulation of synaptic transmission, cholinergic [GO:0032224]; is a type of positive regulation of amine transport [GO:0051954]; positively regulates GO:0014055 Sources: GOC:ef